2-dehydropantolactone reductase (B-specific) activity [GO:0019141] (molecular function) Definition: Catalysis of the reaction: (R)-pantolactone + NADP+ = 2-dehydropantolactone + NADPH + H+. The reaction is B-specific (i.e. the pro-S hydrogen is transferred from the 4-position of reduced nicotinamide cofactor) with respect to NADP+. Sources: EC:1.1.1.214 Also known as: 2-ketopantoyl lactone reductase activity, 2-oxopantoyl lactone reductase, ketopantoyl lactone reductase activity, 2-dehydropantoyl-lactone reductase (B-specific) activity, (R)-pantolactone:NADP+ oxidoreductase (B-specific) Relationships: is a type of 2-dehydropantolactone reductase activity [GO:0036441]